{
  "term_id": "GO:0003723",
  "gene_name": "Interferon-induced protein with tetratricopeptide repeats 1",
  "term_label": "RNA binding",
  "gene_symbol": "IFIT1",
  "gene": "UniProtKB:P09914"
}